{
  "term_id": "GO:0008284",
  "gene": "UniProtKB:P21583",
  "term_label": "positive regulation of cell population proliferation",
  "gene_name": "Kit ligand",
  "gene_symbol": "KITLG"
}